{
  "term_label": "Wnt-protein binding",
  "gene_symbol": "FZD2",
  "term_id": "GO:0017147",
  "gene_name": "Frizzled-2",
  "gene": "UniProtKB:Q14332"
}